{
  "gene_symbol": "MKI67",
  "gene_name": "Proliferation marker protein Ki-67",
  "term_label": "chromosome segregation",
  "gene": "UniProtKB:P46013",
  "term_id": "GO:0007059"
}